{
  "term_id": "GO:0045095",
  "gene_name": "Keratin, type I cuticular Ha6",
  "term_label": "keratin filament",
  "gene": "UniProtKB:O76013",
  "gene_symbol": "KRT36"
}